{
  "term_label": "B cell activation involved in immune response",
  "gene_symbol": "IFNA14",
  "gene_name": "Interferon alpha-14",
  "term_id": "GO:0002312",
  "gene": "UniProtKB:P01570"
}